{
  "term_label": "cell population proliferation",
  "term_id": "GO:0008283",
  "gene_name": "Insulin-like growth factor I",
  "gene": "UniProtKB:P05019",
  "gene_symbol": "IGF1"
}